{
  "gene_symbol": "FGD6",
  "term_id": "GO:0005085",
  "gene": "UniProtKB:Q6ZV73",
  "gene_name": "FYVE, RhoGEF and PH domain-containing protein 6",
  "term_label": "guanyl-nucleotide exchange factor activity"
}